S-adenosylmethionine catabolic process [GO:0050843] (biological process) Also known as: S-adenosyl methionine catabolic process, S-adenosyl methionine catabolism, S-adenosylmethionine breakdown, S-adenosylmethionine catabolism, S-adenosylmethionine degradation, SAM catabolic process Relationships: is a type of sulfur compound catabolic process [GO:0044273]; is a type of S-adenosylmethionine metabolic process [GO:0046500] Sources: GOC:ai Definition: The chemical reactions and pathways resulting in the breakdown of S-adenosylmethionine, S-(5'-adenosyl)-L-methionine, an important intermediate in one-carbon metabolism.